{
  "gene_symbol": "IGHA2",
  "term_id": "GO:0003823",
  "gene": "UniProtKB:P01877",
  "term_label": "antigen binding",
  "gene_name": "Immunoglobulin heavy constant alpha 2"
}